{
  "term_label": "SAGA complex",
  "gene": "UniProtKB:Q14CW9",
  "term_id": "GO:0000124",
  "gene_name": "Ataxin-7-like protein 3",
  "gene_symbol": "ATXN7L3"
}